{
  "term_label": "Unknown cellular component",
  "gene_symbol": "TRIM65",
  "gene_name": "E3 ubiquitin-protein ligase TRIM65",
  "term_id": "UNKNOWN:0003",
  "gene": "UniProtKB:Q6PJ69"
}